{
  "term_id": "GO:0045055",
  "gene": "UniProtKB:Q15907",
  "gene_name": "Ras-related protein Rab-11B",
  "term_label": "regulated exocytosis",
  "gene_symbol": "RAB11B"
}